{
  "gene_symbol": "SMOC1",
  "term_label": "heparin binding",
  "term_id": "GO:0008201",
  "gene": "UniProtKB:Q9H4F8",
  "gene_name": "SPARC-related modular calcium-binding protein 1"
}